prostaglandin-E synthase activity [GO:0050220] (molecular function) Definition: Catalysis of the reaction: prostaglandin H(2) = prostaglandin E(2). Relationships: is a type of intramolecular oxidoreductase activity [GO:0016860] Sources: EC:5.3.99.3, RHEA:12893 Also known as: (5Z,13E)-(15S)-9alpha,11alpha-epidioxy-15-hydroxyprosta-5,13-dienoate E-isomerase activity, PGE isomerase activity, PGE2 isomerase activity, PGH-PGE isomerase activity, Prostaglandin-H(2) E-isomerase activity, endoperoxide isomerase activity, prostaglandin H-E isomerase activity, prostaglandin R-prostaglandin E isomerase activity, prostaglandin endoperoxide E isomerase activity, prostaglandin endoperoxide E2 isomerase activity, prostaglandin-H2 E-isomerase activity